{
  "gene_name": "Nuclear pore complex protein Nup155",
  "gene": "UniProtKB:O75694",
  "term_id": "GO:0006606",
  "gene_symbol": "NUP155",
  "term_label": "protein import into nucleus"
}